{
  "gene_name": "Zinc finger protein 264",
  "term_id": "GO:0000981",
  "gene": "UniProtKB:O43296",
  "term_label": "DNA-binding transcription factor activity, RNA polymerase II-specific",
  "gene_symbol": "ZNF264"
}